{
  "term_label": "chloride transmembrane transport",
  "gene": "UniProtKB:Q9BXS9",
  "term_id": "GO:1902476",
  "gene_symbol": "SLC26A6",
  "gene_name": "Solute carrier family 26 member 6"
}